{
  "gene_symbol": "IMPA2",
  "gene": "UniProtKB:O14732",
  "term_label": "inositol metabolic process",
  "term_id": "GO:0006020",
  "gene_name": "Inositol monophosphatase 2"
}